cellular response to environmental stimulus [GO:0104004] (biological process) Definition: Any process that results in a change in state or activity of a cell (in terms of movement, secretion, enzyme production, gene expression, etc.) as a result of an environmental stimulus. Sources: GOC:dos Relationships: is_a cellular response to stimulus [GO:0051716] Subtypes: cellular response to abiotic stimulus [GO:0071214]